trypanothione synthase activity [GO:0047479] (molecular function) Sources: EC:6.3.1.9, MetaCyc:6.3.1.9-RXN Also known as: TSR synthetase activity, glutathionylspermidine:glutathione ligase (ADP-forming) Definition: Catalysis of the reaction: reduced glutathione + glutathionylspermidine + ATP = trypanothione + ADP + phosphate. Relationships: is a type of acid-ammonia (or amide) ligase activity [GO:0016880]